protein heterotetramerization [GO:0051290] (biological process) Sources: GOC:go_curators Relationships: is a type of GO:0051262; is a type of protein heterooligomerization [GO:0051291] Definition: The formation of a protein heterotetramer, a macromolecular structure consisting of four noncovalently associated subunits, of which not all are identical. Also known as: protein heterotetramer assembly, protein heterotetramer biosynthesis, protein heterotetramer biosynthetic process, protein heterotetramer formation